2-aminobutanoate transaminase activity [GO:0120554] (MF) Definition: Catalysis of the reaction: (2S)-2-aminobutanoate + 2-oxoglutarate = 2-oxobutanoate + L-glutamate. References: PMID:27827456 Sources: RHEA:70223 Relationships: is a type of transaminase activity [GO:0008483]